{
  "gene": "UniProtKB:Q9UHX1",
  "gene_name": "Poly(U)-binding-splicing factor PUF60",
  "term_label": "alternative mRNA splicing, via spliceosome",
  "term_id": "GO:0000380",
  "gene_symbol": "PUF60"
}